ATP-dependent protein disaggregase activity [GO:0140545] (molecular function) Definition: An ATP-dependent molecular chaperone activity that mediates the solubilization of ordered protein aggregates. Also known as: protein disaggregase activity, protein unfoldase activity References: PMID:26312418 Relationships: is a type of ATP-dependent activity [GO:0140657]; is a type of protein-containing complex destabilizing activity [GO:0140776]; has part GO:0005515